negative regulation of respiratory burst [GO:0060268] (biological process) Subtypes: GO:0060266 Relationships: is a type of negative regulation of metabolic process [GO:0009892]; is a type of GO:0060263; negatively regulates respiratory burst [GO:0045730] Sources: GOC:dph, GOC:tb Definition: Any process that decreases the rate frequency or extent of a phase of elevated metabolic activity, during which oxygen consumption increases; this leads to the production, by an NADH dependent system, of hydrogen peroxide (H2O2), superoxide anions and hydroxyl radicals.